{
  "term_label": "nucleolus",
  "gene": "UniProtKB:Q63HN8",
  "gene_name": "E3 ubiquitin-protein ligase RNF213",
  "gene_symbol": "RNF213",
  "term_id": "GO:0005730"
}